{
  "gene": "UniProtKB:C9J202",
  "term_label": "mannosyltransferase activity",
  "gene_name": "Putative glycosyltransferase ALG1L2",
  "term_id": "GO:0000030",
  "gene_symbol": "ALG1L2"
}